{
  "term_id": "GO:0031507",
  "gene_symbol": "LMNB2",
  "term_label": "heterochromatin formation",
  "gene": "UniProtKB:Q03252",
  "gene_name": "Lamin-B2"
}